11-cis-retinal 3,4-desaturase activity [GO:0061899] (molecular function) Definition: Catalysis of the reaction: 11-cis-retinal + 2 H+ + O2 + 2 reduced [adrenodoxin] = 11-cis-3,4-didehydro-retinal + 2 H2O + 2 oxidized [adrenodoxin]. Relationships: is a type of oxidoreductase activity, acting on paired donors, with incorporation or reduction of molecular oxygen [GO:0016705] References: PMID:27059013